{
  "term_id": "UNKNOWN:0001",
  "term_label": "Unknown molecular function",
  "gene_symbol": "SDCBP2",
  "gene_name": "Syntenin-2",
  "gene": "UniProtKB:Q9H190"
}